{
  "gene": "UniProtKB:F5H094",
  "term_label": "sodium-independent organic anion transport",
  "term_id": "GO:0043252",
  "gene_symbol": "SLCO1B3-SLCO1B7",
  "gene_name": "SLCO1B3-SLCO1B7 readthrough transcript protein"
}